Prp19 complex [GO:0000974] (cellular component) Also known as: MOS4-Associated Complex, Prp19/CDC5 complex, nineteen complex, NTC Definition: A protein complex consisting of Prp19 and associated proteins that is involved in the transition from the precatalytic spliceosome to the activated form that catalyzes step 1 of splicing, and which remains associated with the spliceosome through the second catalytic step. It is widely conserved, found in both yeast and mammals, though the exact composition varies. In S. cerevisiae, it contains Prp19p, Ntc20p, Snt309p, Isy1p, Syf2p, Cwc2p, Prp46p, Clf1p, Cef1p, and Syf1p. References: PMID:16540691, PMID:19239890 Sources: GOC:krc Relationships: is_a GO:0032991